{
  "gene_symbol": "SLC38A5",
  "term_id": "GO:0089709",
  "term_label": "L-histidine transmembrane transport",
  "gene_name": "Sodium-coupled neutral amino acid transporter 5",
  "gene": "UniProtKB:Q8WUX1"
}